type 1 somatostatin receptor binding [GO:0031878] (molecular function) Also known as: type 1 somatostatin receptor ligand Definition: Binding to a type 1 somatostatin receptor. Sources: GOC:mah, GOC:nln Relationships: is a type of somatostatin receptor binding [GO:0031877]